{
  "term_label": "nucleus",
  "gene_symbol": "HOXA3",
  "gene": "UniProtKB:O43365",
  "gene_name": "Homeobox protein Hox-A3",
  "term_id": "GO:0005634"
}